{
  "term_id": "GO:0005615",
  "gene_name": "Fibroblast growth factor 3",
  "gene": "UniProtKB:P11487",
  "gene_symbol": "FGF3",
  "term_label": "extracellular space"
}